{
  "term_label": "calcium ion binding",
  "gene_symbol": "S100A10",
  "gene_name": "Protein S100-A10",
  "gene": "UniProtKB:P60903",
  "term_id": "GO:0005509"
}